{
  "term_id": "GO:0002476",
  "term_label": "antigen processing and presentation of endogenous peptide antigen via MHC class Ib",
  "gene_symbol": "HLA-A",
  "gene": "UniProtKB:P04439",
  "gene_name": "HLA class I histocompatibility antigen, A alpha chain"
}